{
  "gene": "UniProtKB:P50416",
  "term_id": "GO:0005739",
  "term_label": "mitochondrion",
  "gene_symbol": "CPT1A",
  "gene_name": "Carnitine O-palmitoyltransferase 1, liver isoform"
}